{
  "term_id": "GO:0005634",
  "gene_symbol": "GON4L",
  "gene": "UniProtKB:Q3T8J9",
  "gene_name": "GON-4-like protein",
  "term_label": "nucleus"
}